aminotriazole transport [GO:0015899] (biological process) Relationships: is a type of GO:0071705 Definition: The directed movement of aminotriazole into, out of or within a cell, or between cells, by means of some agent such as a transporter or pore. Aminotriazole is an effective weed killer that also possesses some antithyroid activity. Sources: GOC:curators